{
  "term_label": "plasma membrane",
  "term_id": "GO:0005886",
  "gene_name": "Olfactory receptor 4M1",
  "gene_symbol": "OR4M1",
  "gene": "UniProtKB:Q8NGD0"
}